{
  "term_label": "Unknown molecular function",
  "gene_name": "Protogenin",
  "gene": "UniProtKB:Q2VWP7",
  "gene_symbol": "PRTG",
  "term_id": "UNKNOWN:0001"
}